serine phosphorylation of STAT protein [GO:0042501] (biological process) Definition: The process of introducing a phosphate group to a serine residue of a STAT (Signal Transducer and Activator of Transcription) protein. Relationships: is a type of peptidyl-serine phosphorylation [GO:0018105]; is part of regulation of receptor signaling pathway via JAK-STAT [GO:0046425] Regulation: regulated by GO:0033139; negatively regulated by negative regulation of peptidyl-serine phosphorylation of STAT protein [GO:0033140]; positively regulated by positive regulation of peptidyl-serine phosphorylation of STAT protein [GO:0033141] Also known as: serine phosphorylation of STAT3 protein References: PMID:10918594 Sources: GOC:jl